{
  "term_id": "UNKNOWN:0001",
  "term_label": "Unknown molecular function",
  "gene": "UniProtKB:Q9H0C1",
  "gene_name": "Zinc finger MYND domain-containing protein 12",
  "gene_symbol": "ZMYND12"
}